{
  "term_label": "purine nucleotide biosynthetic process",
  "gene_symbol": "PRPSAP2",
  "gene_name": "Phosphoribosyl pyrophosphate synthase-associated protein 2",
  "term_id": "GO:0006164",
  "gene": "UniProtKB:O60256"
}